{
  "gene": "UniProtKB:Q9Y4G6",
  "term_id": "GO:0005886",
  "term_label": "plasma membrane",
  "gene_name": "Talin-2",
  "gene_symbol": "TLN2"
}